{
  "gene_name": "Nuclear protein MDM1",
  "gene": "UniProtKB:Q8TC05",
  "term_id": "UNKNOWN:0003",
  "term_label": "Unknown cellular component",
  "gene_symbol": "MDM1"
}